{
  "term_id": "GO:0006915",
  "term_label": "apoptotic process",
  "gene_symbol": "BNIP2",
  "gene": "UniProtKB:Q12982",
  "gene_name": "BCL2_adenovirus E1B 19 kDa protein-interacting protein 2"
}